polyprenol catabolic process [GO:0016095] (biological process) Sources: GOC:go_curators, Wikipedia:Polyprenol Also known as: polyprenol breakdown, polyprenol catabolism, polyprenol degradation Relationships: is a type of isoprenoid catabolic process [GO:0008300]; is a type of polyprenol metabolic process [GO:0016093]; is a type of alcohol catabolic process [GO:0046164] Definition: The chemical reactions and pathways resulting in the breakdown of polyprenols, prenols with more than 4 isoprenoid residues, which may be all-trans, or a mixture of cis and trans. Subtypes: farnesol catabolic process [GO:0016488], geraniol catabolic process [GO:1903447]